homogentisate geranylgeranyltransferase activity [GO:0010356] (molecular function) References: PMID:16989822 Sources: EC:2.5.1.116, GOC:pz Relationships: is a type of homogentisate prenyltransferase activity [GO:0010354] Definition: Catalysis of the reaction: (2E,6E,10E)-geranylgeranyl diphosphate + H+ + homogentisate = 6-geranylgeranyl-2-methylbenzene-1,4-diol + CO2 + diphosphate. Also known as: HGGT activity, homogentisate geranylgeranyl transferase activity